{
  "gene_symbol": "TLE5",
  "gene_name": "TLE family member 5",
  "term_label": "Unknown biological process",
  "term_id": "UNKNOWN:0002",
  "gene": "UniProtKB:Q08117"
}